regulation of synaptic scaling [GO:0150092] (BP) Definition: A process that modulates synaptic scaling. Synaptic scaling is a form of synaptic plasticity, which entails uniform adjustments in the strength of all synapses on a cell in response to prolonged changes in the electrical activity of the cell. References: PMID:14630218, PMID:14735113, PMID:16547515 Sources: GOC:aruk, GOC:bc Relationships: is a type of regulation of synaptic plasticity [GO:0048167] Also known as: homeostatic synaptic scaling, regulation of homeostatic synaptic scaling